{
  "term_id": "UNKNOWN:0003",
  "gene": "UniProtKB:Q8WWR9",
  "term_label": "Unknown cellular component",
  "gene_name": "Pancreatic progenitor cell differentiation and proliferation factor-like protein",
  "gene_symbol": "PPDPFL"
}